{
  "gene": "UniProtKB:Q7RTU5",
  "term_id": "GO:0006357",
  "term_label": "regulation of transcription by RNA polymerase II",
  "gene_name": "Achaete-scute homolog 5",
  "gene_symbol": "ASCL5"
}